{
  "gene_name": "Immunoglobulin kappa variable 3_OR2-268 (non-functional) (Fragment)",
  "gene_symbol": "IGKV3OR2-268",
  "gene": "UniProtKB:A0A0C4DH90",
  "term_label": "immune response",
  "term_id": "GO:0006955"
}